calcium-dependent cell-matrix adhesion [GO:0016340] (biological process) Relationships: is a type of cell-matrix adhesion [GO:0007160] Definition: The binding of a cell to the extracellular matrix via adhesion molecules that require the presence of calcium for the interaction. Sources: GOC:hb